{
  "gene_symbol": "FKBP2",
  "term_label": "endoplasmic reticulum",
  "gene_name": "Peptidyl-prolyl cis-trans isomerase FKBP2",
  "gene": "UniProtKB:P26885",
  "term_id": "GO:0005783"
}